alphav-beta3 integrin-IGF-1-IGF1R complex [GO:0035867] (cellular component) Relationships: is a type of plasma membrane protein complex [GO:0098797] References: PMID:19578119 Sources: GOC:BHF, GOC:ebc Definition: A protein complex that consists of an alphav-beta3 integrin complex bound to insulin-like growth factor-1 (IGF-1) and type I insulin-like growth factor receptor (IGF1R). IGF1R is a heterotetramer that consists of two alpha-subunits and two beta-subunits.